{
  "gene_name": "V-type proton ATPase 116 kDa subunit a 2",
  "gene": "UniProtKB:Q9Y487",
  "gene_symbol": "ATP6V0A2",
  "term_id": "GO:0046961",
  "term_label": "proton-transporting ATPase activity, rotational mechanism"
}